{
  "term_label": "DNA-binding transcription factor activity, RNA polymerase II-specific",
  "term_id": "GO:0000981",
  "gene_symbol": "ETV5",
  "gene": "UniProtKB:P41161",
  "gene_name": "ETS translocation variant 5"
}